{
  "term_label": "phospholipid homeostasis",
  "gene_symbol": "ANGPTL3",
  "term_id": "GO:0055091",
  "gene_name": "Angiopoietin-related protein 3",
  "gene": "UniProtKB:Q9Y5C1"
}